{
  "term_label": "zinc ion binding",
  "gene_symbol": "SEC24C",
  "term_id": "GO:0008270",
  "gene_name": "Protein transport protein Sec24C",
  "gene": "UniProtKB:P53992"
}